{
  "term_label": "cytoplasm",
  "gene": "UniProtKB:Q96PC2",
  "term_id": "GO:0005737",
  "gene_symbol": "IP6K3",
  "gene_name": "Inositol hexakisphosphate kinase 3"
}